{
  "term_id": "UNKNOWN:0003",
  "gene": "UniProtKB:Q9BV20",
  "term_label": "Unknown cellular component",
  "gene_symbol": "MRI1",
  "gene_name": "Methylthioribose-1-phosphate isomerase"
}